{
  "gene_symbol": "C2orf50",
  "gene": "UniProtKB:Q96LR7",
  "gene_name": "Uncharacterized protein C2orf50",
  "term_label": "Unknown biological process",
  "term_id": "UNKNOWN:0002"
}